{
  "gene": "UniProtKB:Q8WU20",
  "term_label": "fibroblast growth factor receptor signaling pathway",
  "term_id": "GO:0008543",
  "gene_symbol": "FRS2",
  "gene_name": "Fibroblast growth factor receptor substrate 2"
}